{
  "gene_symbol": "CRISP3",
  "gene_name": "Cysteine-rich secretory protein 3",
  "gene": "UniProtKB:P54108",
  "term_label": "Unknown molecular function",
  "term_id": "UNKNOWN:0001"
}